{
  "gene": "UniProtKB:P56704",
  "gene_symbol": "WNT3A",
  "term_label": "frizzled binding",
  "term_id": "GO:0005109",
  "gene_name": "Protein Wnt-3a"
}